phosphorylase kinase regulator activity [GO:0008607] (MF) Relationships: is a type of GO:0019887; regulates phosphorylase kinase activity [GO:0004689] Sources: GOC:curators Also known as: phosphorylase kinase, intrinsic regulator activity Definition: Modulation of the activity of the enzyme phosphorylase kinase.